cytosolic DNA-directed RNA polymerase complex [GO:0000345] (cellular component) References: PMID:11158566 Relationships: is_a DNA-directed RNA polymerase complex [GO:0000428]; is part of GO:0005829 Definition: The eubacterial DNA-directed RNA polymerase is a multisubunit complex with a core composed of the essential subunits beta-prime, beta, and two copies of alpha and a fifth nonessential subunit called omega. An additional subunit, a sigma factor, is required for promoter recognition and specificity.